{
  "term_id": "GO:0042500",
  "gene_symbol": "PSEN2",
  "term_label": "aspartic endopeptidase activity, intramembrane cleaving",
  "gene_name": "Presenilin-2",
  "gene": "UniProtKB:P49810"
}